negative regulation of locomotion [GO:0040013] (biological process) Sources: GOC:go_curators Also known as: down regulation of locomotion, down-regulation of locomotion, downregulation of locomotion, inhibition of locomotion Relationships: is a type of GO:0040012; is a type of negative regulation of biological process [GO:0048519]; negatively regulates GO:0040011 Definition: Any process that stops, prevents, or reduces the frequency, rate or extent of locomotion of a cell or organism. Subtypes: negative regulation of chemotaxis [GO:0050922], negative regulation of locomotion involved in locomotory behavior [GO:0090327], negative regulation of forward locomotion [GO:1905849], negative regulation of backward locomotion [GO:1905851], GO:2000146